{
  "term_label": "metalloendopeptidase activity",
  "gene_name": "Stromelysin-1",
  "gene": "UniProtKB:P08254",
  "term_id": "GO:0004222",
  "gene_symbol": "MMP3"
}